{
  "gene_name": "Integrin alpha-9",
  "term_id": "GO:0098609",
  "gene": "UniProtKB:Q13797",
  "term_label": "cell-cell adhesion",
  "gene_symbol": "ITGA9"
}